{
  "gene_name": "Complement C3",
  "term_id": "GO:0006956",
  "gene_symbol": "C3",
  "term_label": "complement activation",
  "gene": "UniProtKB:P01024"
}